positive regulation of small intestine smooth muscle contraction [GO:1904349] (BP) References: PMID:11991626 Sources: GOC:TermGenie, GO_REF:0000058 Also known as: up regulation of small intestine smooth muscle contraction, up-regulation of small intestine smooth muscle contraction, upregulation of small intestine smooth muscle contraction, activation of small intestine smooth muscle contraction Relationships: is a type of positive regulation of gastro-intestinal system smooth muscle contraction [GO:1904306]; is a type of regulation of small intestine smooth muscle contraction [GO:1904347]; positively regulates GO:1990770 Definition: Any process that activates or increases the frequency, rate or extent of small intestine smooth muscle contraction.